oxidoreductase activity, acting on NAD(P)H as acceptor [GO:0016652] (molecular function) Sources: EC:1.6.1.- Definition: Catalysis of an oxidation-reduction (redox) reaction in which NADH or NADPH acts as a hydrogen or electron donor and reduces NAD+ or NADP. Also known as: oxidoreductase activity, acting on NAD or NADPH, NAD or NADP as acceptor Subtypes: NAD(P)+ transhydrogenase (Si-specific) activity [GO:0003957] Relationships: is a type of oxidoreductase activity, acting on NAD(P)H [GO:0016651]